cleistothecium formation [GO:0062248] (biological process) Relationships: is a type of anatomical structure formation involved in morphogenesis [GO:0048646]; is part of cleistothecium development [GO:0070791] Definition: The process of producing a cleistothecium, a closed sexual fruiting body that contains ascospores in linear asci. Cleistothecia are present in some filamentous Ascomycete fungi such as members of the genera Aspergillus and Emericella. References: PMID:20348388, PMID:28889020, PMID:30410052